vibrational conductance of sound to the inner ear [GO:0055127] (biological process) Sources: GOC:mh Relationships: is a type of multicellular organismal process [GO:0032501]; is part of sensory perception of sound [GO:0007605] Definition: The transmission of vibrations via ossicles to the inner ear.